{
  "gene_symbol": "PRF1",
  "gene": "UniProtKB:P14222",
  "term_label": "defense response to virus",
  "gene_name": "Perforin-1",
  "term_id": "GO:0051607"
}